{
  "gene": "UniProtKB:Q6DKK2",
  "term_id": "UNKNOWN:0001",
  "gene_symbol": "TTC19",
  "gene_name": "Tetratricopeptide repeat protein 19, mitochondrial",
  "term_label": "Unknown molecular function"
}